{
  "term_label": "RNA polymerase II cis-regulatory region sequence-specific DNA binding",
  "gene_symbol": "ZNF195",
  "term_id": "GO:0000978",
  "gene_name": "Zinc finger protein 195",
  "gene": "UniProtKB:O14628"
}